{
  "gene_name": "Protein WFDC9",
  "gene": "UniProtKB:Q8NEX5",
  "gene_symbol": "WFDC9",
  "term_id": "GO:0005615",
  "term_label": "extracellular space"
}